{
  "gene_symbol": "EBF2",
  "gene_name": "Transcription factor COE2",
  "gene": "UniProtKB:Q9HAK2",
  "term_label": "Unknown cellular component",
  "term_id": "UNKNOWN:0003"
}